RNA polymerase I cis-regulatory region sequence-specific DNA binding [GO:0001165] (molecular function) Also known as: RNA polymerase I enhancer sequence-specific DNA binding, RNA polymerase I upstream control element sequence-specific DNA binding, RNA polymerase I upstream element sequence-specific DNA binding References: PMID:12865296, PMID:14969726, PMID:8057832 Sources: GOC:txnOH Definition: Binding to a specific upstream regulatory DNA sequence (transcription factor recognition sequence or binding site) located in cis relative to the transcription start site (i.e., on the same strand of DNA) of a gene transcribed by RNA polymerase I. RNA polymerase I elements are referred to either enhancers or upstream control element (UCE, or alternately referred to as the upstream element). Relationships: is a type of RNA polymerase I transcription regulatory region sequence-specific DNA binding [GO:0001163]